{
  "gene": "UniProtKB:O43557",
  "gene_name": "Tumor necrosis factor ligand superfamily member 14",
  "gene_symbol": "TNFSF14",
  "term_id": "GO:0005615",
  "term_label": "extracellular space"
}